elongation factor-2 kinase activity [GO:0004686] (molecular function) Definition: Catalysis of the reaction: ATP + [elongation factor 2] = ADP + [elongation factor 2] phosphate. Also known as: eEF-2 kinase activity, ATP:elongation factor 2 phosphotransferase activity, Ca/CaM-kinase III activity, CaM kinase III activity, EF2K, STK19, calmodulin-dependent protein kinase III activity, eEF2 kinase activity, eEF2K, elongation factor 2 kinase activity, eukaryotic elongation factor 2 kinase activity Relationships: is a type of GO:0004683 Sources: EC:2.7.11.20, MetaCyc:2.7.11.20-RXN Regulation: regulated by eukaryotic elongation factor-2 kinase regulator activity [GO:0042556]; positively regulated by eukaryotic elongation factor-2 kinase activator activity [GO:0042557]